{
  "gene_name": "Proto-oncogene tyrosine-protein kinase Src",
  "term_id": "GO:0005886",
  "gene_symbol": "SRC",
  "term_label": "plasma membrane",
  "gene": "UniProtKB:P12931"
}